{
  "gene": "UniProtKB:Q15555",
  "term_label": "microtubule organizing center",
  "gene_symbol": "MAPRE2",
  "gene_name": "Microtubule-associated protein RP_EB family member 2",
  "term_id": "GO:0005815"
}